{
  "term_label": "regulation of DNA-templated transcription",
  "gene_symbol": "MYCBP",
  "gene": "UniProtKB:Q99417",
  "gene_name": "c-Myc-binding protein",
  "term_id": "GO:0006355"
}